negative regulation of hyaluranon cable assembly [GO:1900105] (biological process) Sources: GOC:TermGenie, GOC:yaf Definition: Any process that stops, prevents or reduces the frequency, rate or extent of hyaluranon cable assembly. Relationships: is_a negative regulation of cellular component organization [GO:0051129]; is a type of regulation of hyaluranon cable assembly [GO:1900104]; negatively regulates hyaluranon cable assembly [GO:0036118] Also known as: down regulation of HA cable assembly, down regulation of hyaluranon cable assembly, down-regulation of HA cable assembly, down-regulation of hyaluranon cable assembly, downregulation of HA cable assembly, downregulation of hyaluranon cable assembly, inhibition of HA cable assembly, negative regulation of HA cable assembly, inhibition of hyaluranon cable assembly